{
  "term_id": "GO:0005886",
  "gene_symbol": "TRBV5-4",
  "term_label": "plasma membrane",
  "gene": "UniProtKB:A0A0C4DH59",
  "gene_name": "T cell receptor beta variable 5-4"
}